{
  "term_label": "basal RNA polymerase II transcription machinery binding",
  "gene_symbol": "LLPH",
  "gene": "UniProtKB:Q9BRT6",
  "gene_name": "Protein LLP homolog",
  "term_id": "GO:0001099"
}